Rho-dependent protein serine/threonine kinase activity [GO:0072518] (molecular function) Relationships: is a type of protein serine/threonine kinase activity [GO:0004674] References: PMID:12778124, PMID:20230755 Sources: GOC:ecd Note: This reaction requires binding of the GTPase Rho. Also known as: ROCK kinase activity, Rho-associated protein kinase activity Regulation: regulated by regulation of Rho-dependent protein serine/threonine kinase activity [GO:2000298]; RO_0002212 by negative regulation of Rho-dependent protein serine/threonine kinase activity [GO:2000299] Definition: Rho GTPase-dependent catalysis of the reaction: ATP + a protein = ADP + a phosphoprotein.